regulation of transcription by RNA polymerase V [GO:1904279] (biological process) Relationships: is a type of regulation of DNA-templated transcription [GO:0006355]; regulates transcription by RNA polymerase V [GO:0001060] Also known as: regulation of transcription from RNA pol V promoter, regulation of transcription from RNA polymerase V promoter References: PMID:24726328 Sources: GOC:TermGenie, GO_REF:0000058 Subtypes: negative regulation of transcription by RNA polymerase V [GO:1904280], positive regulation of transcription by RNA polymerase V [GO:1904281] Definition: Any process that modulates the frequency, rate or extent of transcription mediated by RNA polymerase V.